{
  "term_id": "GO:0071230",
  "gene": "UniProtKB:Q9UHA4",
  "term_label": "cellular response to amino acid stimulus",
  "gene_name": "Ragulator complex protein LAMTOR3",
  "gene_symbol": "LAMTOR3"
}